organ growth [GO:0035265] (BP) Definition: The increase in size or mass of an organ. Organs are commonly observed as visibly distinct structures, but may also exist as loosely associated clusters of cells that function together as to perform a specific function. Sources: GOC:bf, ISBN:0471245208, ISBN:0721662544 Relationships: is_a GO:0032501; is_a developmental growth [GO:0048589] Subtypes: heart growth [GO:0060419], GO:0060437, prostate gland growth [GO:0060736], bone growth [GO:0098868] Regulation: regulated by regulation of organ growth [GO:0046620]; negatively regulated by negative regulation of organ growth [GO:0046621]; positively regulated by positive regulation of organ growth [GO:0046622]